centralspindlin complex [GO:0097149] (cellular component) Relationships: is a type of intracellular protein-containing complex [GO:0140535]; is part of mitotic spindle [GO:0072686] References: PMID:11782313, PMID:16236794 Sources: GOC:ans Definition: A heterotetrameric protein complex playing a key role in the formation of the central spindle in mitosis. Made up of two molecules each of a mitotic kinesin (ZEN-4 in Caenorhabditis elegans or MKLP1 in mammals) and of two molecules each of a GTPase activating protein (GAP) factor (CYK-4 in Caenorhabditis elegans or MgcRacGAP in mammals).